{
  "gene_symbol": "DRAXIN",
  "gene": "UniProtKB:Q8NBI3",
  "term_id": "GO:0021516",
  "gene_name": "Draxin",
  "term_label": "dorsal spinal cord development"
}